{
  "gene_symbol": "ACSS3",
  "term_id": "UNKNOWN:0002",
  "gene_name": "Acyl-CoA synthetase short-chain family member 3, mitochondrial",
  "gene": "UniProtKB:Q9H6R3",
  "term_label": "Unknown biological process"
}